{
  "gene_name": "Collagen and calcium-binding EGF domain-containing protein 1",
  "gene": "UniProtKB:Q6UXH8",
  "term_id": "GO:0001946",
  "gene_symbol": "CCBE1",
  "term_label": "lymphangiogenesis"
}